{
  "term_id": "GO:0019901",
  "gene": "UniProtKB:Q9Y3I1",
  "gene_symbol": "FBXO7",
  "gene_name": "F-box only protein 7",
  "term_label": "protein kinase binding"
}